{
  "gene_name": "Ubiquitin-conjugating enzyme E2 J2",
  "gene": "UniProtKB:Q8N2K1",
  "term_label": "ubiquitin conjugating enzyme activity",
  "term_id": "GO:0061631",
  "gene_symbol": "UBE2J2"
}